{
  "term_id": "GO:0005634",
  "gene": "UniProtKB:Q09FC8",
  "term_label": "nucleus",
  "gene_name": "Zinc finger protein 415",
  "gene_symbol": "ZNF415"
}